peptidyl-tyrosine hydroxylation [GO:0018336] (BP) Definition: The hydroxylation of peptidyl-tyrosine to form peptidyl-dihydroxyphenylalanine. Sources: GOC:ai Relationships: is a type of protein hydroxylation [GO:0018126]